{
  "gene_name": "T cell receptor alpha joining 12 (Fragment)",
  "gene_symbol": "TRAJ12",
  "term_label": "Unknown cellular component",
  "gene": "UniProtKB:A0A075B6U8",
  "term_id": "UNKNOWN:0003"
}